{
  "term_id": "GO:0005814",
  "gene": "UniProtKB:Q8N3Y1",
  "term_label": "centriole",
  "gene_symbol": "FBXW8",
  "gene_name": "F-box_WD repeat-containing protein 8"
}